lycopene catabolic process [GO:1901176] (biological process) Sources: GOC:TermGenie, GOC:yaf, UniPathway:UPA00803 Relationships: is a type of carotene catabolic process [GO:0016121] Also known as: lycopene breakdown, lycopene catabolism, lycopene degradation Definition: The chemical reactions and pathways resulting in the breakdown of lycopene.